{
  "gene_name": "Trans-Golgi network integral membrane protein 2",
  "gene_symbol": "TGOLN2",
  "term_id": "UNKNOWN:0001",
  "term_label": "Unknown molecular function",
  "gene": "UniProtKB:O43493"
}